phosphoribosylaminoimidazole carboxylase activity [GO:0004638] (molecular function) Sources: EC:4.1.1.21, RHEA:10792 Definition: Catalysis of the reaction: 5-amino-1-(5-phospho-D-ribosyl)imidazole-4-carboxylate + 2 H+ = 5-amino-1-(5-phospho-D-ribosyl)imidazole + CO2. Also known as: 1-(5-phosphoribosyl)-5-amino-4-imidazolecarboxylate carboxy-lyase activity, 5-amino-1-(5-phospho-D-ribosyl)imidazole-4-carboxylate carboxy-lyase [5-amino-1-(5-phospho-D-ribosyl)imidazole-forming], 5-amino-1-(5-phospho-D-ribosyl)imidazole-4-carboxylate carboxy-lyase activity, 5-amino-1-ribosylimidazole 5-phosphate carboxylase activity, 5-phosphoribosyl-5-aminoimidazole carboxylase activity, ADE2, AIR carboxylase activity, class II PurE Relationships: is a type of carboxy-lyase activity [GO:0016831]